{
  "gene_name": "Putative uncharacterized protein GSN-AS1",
  "gene_symbol": "GSN-AS1",
  "term_label": "Unknown cellular component",
  "term_id": "UNKNOWN:0003",
  "gene": "UniProtKB:Q9NRJ2"
}